{
  "gene_name": "TATA-box-binding protein-associated factor 11-like protein 7",
  "gene": "UniProtKB:P0DW12",
  "term_id": "GO:0005669",
  "gene_symbol": "TAF11L7",
  "term_label": "transcription factor TFIID complex"
}